{
  "gene_name": "Hexokinase-2",
  "term_id": "GO:0001678",
  "term_label": "intracellular glucose homeostasis",
  "gene": "UniProtKB:P52789",
  "gene_symbol": "HK2"
}